maintenance of granzyme B location in T cell secretory granule [GO:0033382] (biological process) Sources: GOC:mah Also known as: maintenance of granzyme B localization in T lymphocyte secretory granule, maintenance of granzyme B localization in T-cell secretory granule, maintenance of granzyme B localization in T-lymphocyte secretory granule, maintenance of granzyme B localization in T cell secretory granule Definition: A process in which the protease granyme B is maintained in a secretory granule in a T cell and prevented from moving elsewhere. Relationships: is a type of maintenance of protease location in T cell secretory granule [GO:0033379]; is part of GO:0033380